regulation of bone remodeling [GO:0046850] (biological process) Definition: Any process that modulates the frequency, rate or extent of bone remodeling, the processes of bone formation and resorption that combine to maintain skeletal integrity. Sources: GOC:ai Also known as: regulation of bone remodelling Subtypes: regulation of bone resorption [GO:0045124], negative regulation of bone remodeling [GO:0046851], positive regulation of bone remodeling [GO:0046852] Relationships: is a type of GO:0034103; regulates bone remodeling [GO:0046849]